protein localization to endosome [GO:0036010] (biological process) Also known as: protein localisation in endosome, protein localization in endosome Regulation: RO_0002211 by regulation of protein localization to endosome [GO:1905666]; negatively regulated by negative regulation of protein localization to endosome [GO:1905667]; positively regulated by positive regulation of protein localization to endosome [GO:1905668] Definition: A process in which a protein is transported to, or maintained in, a location within an endosome. Sources: GOC:yaf Relationships: is a type of protein localization to organelle [GO:0033365] Subtypes: neurotransmitter receptor transport, plasma membrane to endosome [GO:0099646], protein localization to early endosome [GO:1902946]